{
  "term_id": "GO:0045987",
  "gene_symbol": "EDN3",
  "term_label": "positive regulation of smooth muscle contraction",
  "gene": "UniProtKB:P14138",
  "gene_name": "Endothelin-3"
}